{
  "term_label": "plasma membrane",
  "gene_name": "Transient receptor potential cation channel subfamily V member 6",
  "gene_symbol": "TRPV6",
  "term_id": "GO:0005886",
  "gene": "UniProtKB:Q9H1D0"
}